{
  "term_label": "Unknown biological process",
  "gene_name": "Superoxide dismutase [Mn], mitochondrial",
  "gene_symbol": "SOD2",
  "term_id": "UNKNOWN:0002",
  "gene": "UniProtKB:P04179"
}